{
  "gene": "UniProtKB:Q96RY5",
  "gene_name": "Protein cramped-like",
  "gene_symbol": "CRAMP1",
  "term_id": "GO:0005634",
  "term_label": "nucleus"
}